benzyl-2-methyl-hydroxybutyrate dehydrogenase activity [GO:0047027] (molecular function) Relationships: is a type of oxidoreductase activity, acting on the CH-OH group of donors, NAD or NADP as acceptor [GO:0016616] Definition: Catalysis of the reaction: benzyl (2R,3S)-2-methyl-3-hydroxybutanoate + NADP+ = benzyl 2-methyl-3-oxobutanoate + H+ + NADPH. Also known as: benzyl 2-methyl-3-hydroxybutyrate dehydrogenase activity, benzyl-(2R,3S)-2-methyl-3-hydroxybutanoate:NADP+ 3-oxidoreductase activity Sources: EC:1.1.1.217, RHEA:16405